{
  "term_label": "nucleosome",
  "term_id": "GO:0000786",
  "gene_symbol": "H2AC17",
  "gene_name": "Histone H2A type 1",
  "gene": "UniProtKB:P0C0S8"
}